{
  "gene": "UniProtKB:Q99593",
  "gene_name": "T-box transcription factor TBX5",
  "term_label": "regulation of transcription by RNA polymerase II",
  "term_id": "GO:0006357",
  "gene_symbol": "TBX5"
}